GMP synthase activity [GO:0003921] (molecular function) Definition: Catalysis of the reaction: ATP + XMP + NH4(+) = AMP + diphosphate + GMP + 2H+. Sources: RHEA:18301 Relationships: is a type of ligase activity, forming carbon-nitrogen bonds [GO:0016879]; is part of GMP synthase (glutamine-hydrolyzing) activity [GO:0003922]